{
  "gene": "UniProtKB:Q9Y5P2",
  "gene_symbol": "CSAG3",
  "term_id": "UNKNOWN:0002",
  "gene_name": "Chondrosarcoma-associated gene 2_3 protein",
  "term_label": "Unknown biological process"
}